{
  "term_label": "plasma membrane",
  "term_id": "GO:0005886",
  "gene_name": "Neuronal membrane glycoprotein M6-a",
  "gene": "UniProtKB:P51674",
  "gene_symbol": "GPM6A"
}